vacuolar acidification [GO:0007035] (biological process) Definition: Any process that reduces the pH of the vacuole, measured by the concentration of the hydrogen ion. Relationships: is a type of GO:0051452 Subtypes: lysosomal lumen acidification [GO:0007042] Sources: GOC:jid